{
  "gene": "UniProtKB:P0C2W7",
  "gene_name": "Cancer_testis antigen family 47 member B1",
  "term_label": "Unknown cellular component",
  "term_id": "UNKNOWN:0003",
  "gene_symbol": "CT47B1"
}